{
  "gene": "UniProtKB:Q6ZN84",
  "term_label": "Unknown biological process",
  "term_id": "UNKNOWN:0002",
  "gene_name": "Coiled-coil domain-containing protein 81",
  "gene_symbol": "CCDC81"
}